{
  "term_label": "positive regulation of Rho protein signal transduction",
  "gene_symbol": "ABRA",
  "term_id": "GO:0035025",
  "gene": "UniProtKB:Q8N0Z2",
  "gene_name": "Actin-binding Rho-activating protein"
}